{
  "gene": "UniProtKB:Q14CS0",
  "gene_name": "UBX domain-containing protein 2B",
  "term_label": "membrane fusion",
  "term_id": "GO:0061025",
  "gene_symbol": "UBXN2B"
}